{
  "gene_symbol": "BAG5",
  "term_label": "protein stabilization",
  "gene": "UniProtKB:Q9UL15",
  "gene_name": "BAG family molecular chaperone regulator 5",
  "term_id": "GO:0050821"
}